{
  "gene_symbol": "CNST",
  "gene_name": "Consortin",
  "term_id": "GO:0071253",
  "gene": "UniProtKB:Q6PJW8",
  "term_label": "connexin binding"
}